{
  "gene_name": "Phospholipid-transporting ATPase IH",
  "term_id": "GO:0005886",
  "gene_symbol": "ATP11A",
  "gene": "UniProtKB:P98196",
  "term_label": "plasma membrane"
}